{
  "gene": "UniProtKB:P35590",
  "term_label": "plasma membrane",
  "gene_symbol": "TIE1",
  "gene_name": "Tyrosine-protein kinase receptor Tie-1",
  "term_id": "GO:0005886"
}